{
  "gene_symbol": "VTI1A",
  "term_id": "GO:0006896",
  "gene": "UniProtKB:Q96AJ9",
  "term_label": "Golgi to vacuole transport",
  "gene_name": "Vesicle transport through interaction with t-SNAREs homolog 1A"
}